{
  "gene_name": "Putative protein SNX29P2",
  "term_id": "UNKNOWN:0002",
  "gene": "UniProtKB:Q8IUI4",
  "term_label": "Unknown biological process",
  "gene_symbol": "SNX29P2"
}